{
  "gene": "UniProtKB:P35606",
  "term_label": "intracellular protein transport",
  "gene_symbol": "COPB2",
  "gene_name": "Coatomer subunit beta'",
  "term_id": "GO:0006886"
}